{
  "gene_name": "Metallothionein-1L",
  "gene": "UniProtKB:Q93083",
  "gene_symbol": "MT1L",
  "term_id": "GO:0071294",
  "term_label": "cellular response to zinc ion"
}